anterior/posterior pattern specification, imaginal disc [GO:0007448] (biological process) Definition: The establishment, maintenance and elaboration of the anterior/posterior axis of the imaginal disc. Imaginal discs are epithelial infoldings in the larvae of holometabolous insects that rapidly develop into adult appendages during metamorphosis from larval to adult form. Relationships: is a type of imaginal disc pattern formation [GO:0007447]; is a type of anterior/posterior pattern specification [GO:0009952] Subtypes: leg disc anterior/posterior pattern formation [GO:0035200], genital disc anterior/posterior pattern formation [GO:0035224], wing disc anterior/posterior pattern formation [GO:0048100] Sources: GOC:bf, ISBN:0879694238